generation of catalytic spliceosome for second transesterification step [GO:0000350] (biological process) Sources: GOC:krc, ISBN:0879695897 Note: Note that this step represents formation of the A2-3 complex (yeast) or the C2 complex (mammalian). Relationships: is_a protein-RNA complex assembly [GO:0022618]; is part of spliceosomal conformational changes to generate catalytic conformation [GO:0000393] Also known as: formation of catalytic spliceosome for second transesterification step, formation of catalytic U12-type spliceosome for second transesterification step, formation of catalytic U2-type spliceosome for second transesterification step, formation of spliceosomal A2-2 complex, formation of spliceosomal C1 complex, spliceosomal A2-3 complex biosynthesis, spliceosomal A2-3 complex formation, spliceosomal C2 complex biosynthesis, spliceosomal C2 complex formation, catalytic spliceosome assembly for second transesterification step, lariat formation, 5'-splice site cleavage Definition: Conformational rearrangement of the spliceosomal complex containing the RNA products from the 1st step of splicing to form the catalytic site for the second step of splicing.